{
  "term_label": "regulation of immune system process",
  "gene_name": "Zinc finger and BTB domain-containing protein 39",
  "gene": "UniProtKB:O15060",
  "gene_symbol": "ZBTB39",
  "term_id": "GO:0002682"
}